{
  "gene_name": "PRAME family member 27",
  "gene_symbol": "PRAMEF27",
  "term_label": "proteasome-mediated ubiquitin-dependent protein catabolic process",
  "gene": "UniProtKB:A3QJZ7",
  "term_id": "GO:0043161"
}